{
  "term_id": "GO:0000981",
  "gene": "UniProtKB:P17017",
  "gene_name": "Zinc finger protein 14",
  "gene_symbol": "ZNF14",
  "term_label": "DNA-binding transcription factor activity, RNA polymerase II-specific"
}